{
  "gene": "UniProtKB:Q8TDC0",
  "term_id": "GO:0030018",
  "term_label": "Z disc",
  "gene_name": "Myozenin-3",
  "gene_symbol": "MYOZ3"
}